{
  "gene_name": "BTB_POZ domain-containing protein KCTD1",
  "term_label": "transcription corepressor activity",
  "term_id": "GO:0003714",
  "gene": "UniProtKB:Q719H9",
  "gene_symbol": "KCTD1"
}